{
  "term_label": "regulation of transcription by RNA polymerase II",
  "gene_symbol": "NFIC",
  "gene_name": "Nuclear factor 1 C-type",
  "gene": "UniProtKB:P08651",
  "term_id": "GO:0006357"
}